{
  "gene_name": "Ribosomal RNA-processing protein 8",
  "gene": "UniProtKB:O43159",
  "term_label": "Unknown molecular function",
  "gene_symbol": "RRP8",
  "term_id": "UNKNOWN:0001"
}